{
  "term_id": "GO:0045664",
  "gene_name": "Zinc finger homeobox protein 3",
  "gene_symbol": "ZFHX3",
  "gene": "UniProtKB:Q15911",
  "term_label": "regulation of neuron differentiation"
}